{
  "term_id": "GO:0003690",
  "gene": "UniProtKB:P16401",
  "gene_symbol": "H1-5",
  "term_label": "double-stranded DNA binding",
  "gene_name": "Histone H1.5"
}